{
  "term_id": "UNKNOWN:0003",
  "gene_symbol": "NPIPA3",
  "gene_name": "Nuclear pore complex-interacting protein family member A3",
  "gene": "UniProtKB:F8WFD2",
  "term_label": "Unknown cellular component"
}